(N-acetylneuraminyl)-galactosylglucosylceramide N-acetylgalactosaminyltransferase activity [GO:0003947] (molecular function) Sources: EC:2.4.1.92 Relationships: is a type of acetylgalactosaminyltransferase activity [GO:0008376] Definition: Catalysis of the reaction: UDP-N-acetyl-D-galactosamine + (N-acetylneuraminyl)-D-galactosyl-D-glucosylceramide = UDP + N-acetyl-D-galactosaminyl-(N-acetylneuraminyl)-D-galactosyl-D-glucosylceramide. Also known as: GM2 synthase activity, GM2/GD2-synthase activity, GalNAc-T activity, UDP acetylgalactosamine-(N-acetylneuraminyl)-D-galactosyl-D-glucosylceramide acetylgalactosaminyltransferase activity, UDP-N-acetyl-D-galactosamine:(N-acetylneuraminyl)-D-galactosyl-D-glucosylceramide N-acetyl-D-galactosaminyltransferase activity, UDP-N-acetyl-D-galactosamine:1-O-[O-(N-acetyl-alpha-neuraminosyl)-(2->3)-O-beta-D-galactopyranosyl-(1->4)-beta-D-glucopyranosyl]-ceramide 1,4-beta-N-acetyl-D-galactosaminyltransferase activity, UDP-N-acetylgalactosamine GM3 N-acetylgalactosaminyltransferase activity, asialo-GM2 synthase activity, beta-1,4N-aetylgalactosaminyltransferase activity, ganglioside GM2 synthase activity, ganglioside GM3 acetylgalactosaminyltransferase activity, uridine diphosphoacetylgalactosamine-acetylneuraminylgalactosylglucosylceramide acetylgalactosaminyltransferase activity, uridine diphosphoacetylgalactosamine-ganglioside GM3 acetylgalactosaminyltransferase activity, uridine diphosphoacetylgalactosamine-hematoside acetylgalactosaminyltransferase activity